{
  "term_id": "GO:0016324",
  "gene_symbol": "SLC17A5",
  "gene": "UniProtKB:Q9NRA2",
  "term_label": "apical plasma membrane",
  "gene_name": "Sialin"
}